{
  "gene": "UniProtKB:Q9P270",
  "gene_symbol": "SLAIN2",
  "term_id": "GO:0035371",
  "term_label": "microtubule plus-end",
  "gene_name": "SLAIN motif-containing protein 2"
}